{
  "gene_symbol": "ARCN1",
  "gene_name": "Coatomer subunit delta",
  "term_label": "retrograde vesicle-mediated transport, Golgi to endoplasmic reticulum",
  "gene": "UniProtKB:P48444",
  "term_id": "GO:0006890"
}